{
  "gene_symbol": "ZBED2",
  "term_id": "GO:0000122",
  "term_label": "negative regulation of transcription by RNA polymerase II",
  "gene": "UniProtKB:Q9BTP6",
  "gene_name": "Zinc finger BED domain-containing protein 2"
}